{
  "gene_name": "GPI mannosyltransferase 2",
  "term_id": "GO:0005789",
  "gene_symbol": "PIGV",
  "term_label": "endoplasmic reticulum membrane",
  "gene": "UniProtKB:Q9NUD9"
}